{
  "gene_symbol": "SLC23A1",
  "gene_name": "Solute carrier family 23 member 1",
  "gene": "UniProtKB:Q9UHI7",
  "term_id": "GO:0016324",
  "term_label": "apical plasma membrane"
}